{
  "term_id": "GO:0001632",
  "gene_symbol": "LTB4R2",
  "gene_name": "Leukotriene B4 receptor 2",
  "term_label": "leukotriene B4 receptor activity",
  "gene": "UniProtKB:Q9NPC1"
}